{
  "gene_name": "T-cell surface glycoprotein CD3 delta chain",
  "term_label": "external side of plasma membrane",
  "gene": "UniProtKB:P04234",
  "gene_symbol": "CD3D",
  "term_id": "GO:0009897"
}